{
  "gene_symbol": "ADGRA2",
  "term_id": "GO:0002040",
  "gene_name": "Adhesion G protein-coupled receptor A2",
  "term_label": "sprouting angiogenesis",
  "gene": "UniProtKB:Q96PE1"
}